{
  "gene_name": "Intermembrane lipid transfer protein VPS13C",
  "term_label": "mitochondrion organization",
  "gene": "UniProtKB:Q709C8",
  "gene_symbol": "VPS13C",
  "term_id": "GO:0007005"
}